{
  "gene": "UniProtKB:Q6UXI9",
  "gene_symbol": "NPNT",
  "term_id": "UNKNOWN:0003",
  "term_label": "Unknown cellular component",
  "gene_name": "Nephronectin"
}